{
  "term_id": "GO:0051082",
  "gene_symbol": "NACA4P",
  "gene_name": "Putative nascent polypeptide-associated complex subunit alpha-like protein",
  "gene": "UniProtKB:Q9BZK3",
  "term_label": "unfolded protein binding"
}